{
  "gene_symbol": "H2BC19P",
  "gene_name": "Putative histone H2B type 2-D",
  "gene": "UniProtKB:Q6DRA6",
  "term_id": "GO:0019731",
  "term_label": "antibacterial humoral response"
}